cerebroside transfer activity [GO:0140340] (molecular function) Definition: Directly binding to a cerebroside and delivering it either to an acceptor molecule or to a specific location. Also known as: cerebroside carrier activity References: PMID:9132017 Relationships: is_a GO:0017089; is a type of ceramide transfer activity [GO:0120017]